{
  "gene_symbol": "LGALS3",
  "term_label": "IgE binding",
  "term_id": "GO:0019863",
  "gene": "UniProtKB:P17931",
  "gene_name": "Galectin-3"
}